galactosylxylosylprotein 3-beta-galactosyltransferase activity [GO:0047220] (molecular function) Sources: EC:2.4.1.134, MetaCyc:2.4.1.134-RXN Definition: Catalysis of the reaction: 4-beta-D-galactosyl-O-beta-D-xylosylprotein + UDP-galactose = 3-beta-D-galactosyl-4-beta-D-galactosyl-O-beta-D-xylosylprotein + UDP. Relationships: is a type of GO:0035250; is a type of GO:0140103 Also known as: UDP-galactose:4-beta-D-galactosyl-O-beta-D-xylosylprotein 3-beta-D-galactosyltransferase activity, UDPgalactose:4-beta-D-galactosyl-O-beta-D-xylosylprotein 3-beta-D-galactosyltransferase activity, galactosyltransferase II activity, uridine diphosphogalactose-galactosylxylose galactosyltransferase activity